carnitine O-octanoyltransferase activity [GO:0008458] (molecular function) Definition: Catalysis of the reaction: (R)-carnitine + octanoyl-CoA = CoA + O-octanoyl-(R)-carnitine. Sources: RHEA:17177 Also known as: easily solubilized mitochondrial carnitine palmitoyltransferase, overt mitochondrial carnitine palmitoyltransferase, carnitine medium-chain acyltransferase activity, medium-chain/long-chain carnitine acyltransferase activity, octanoyl-CoA:L-carnitine O-octanoyltransferase activity Relationships: is a type of GO:0016406